{
  "gene": "UniProtKB:Q9HB66",
  "term_id": "UNKNOWN:0002",
  "gene_name": "Alternative protein MKKS",
  "gene_symbol": "MKKS",
  "term_label": "Unknown biological process"
}